{
  "gene_name": "Putative uncharacterized protein FLJ13197",
  "term_id": "UNKNOWN:0003",
  "gene_symbol": "Q9H8V8",
  "term_label": "Unknown cellular component",
  "gene": "UniProtKB:Q9H8V8"
}